{
  "gene_symbol": "ZNF44",
  "term_id": "GO:0005634",
  "term_label": "nucleus",
  "gene_name": "Zinc finger protein 44",
  "gene": "UniProtKB:P15621"
}